{
  "gene": "UniProtKB:Q5QNW6",
  "gene_name": "Histone H2B type 2-F",
  "term_label": "nucleosome",
  "gene_symbol": "H2BC18",
  "term_id": "GO:0000786"
}